macrophage inflammatory protein-1 gamma production [GO:0071607] (biological process) Regulation: regulated by regulation of macrophage inflammatory protein-1 gamma production [GO:0071646]; negatively regulated by negative regulation of macrophage inflammatory protein-1 gamma production [GO:0071647]; RO_0002213 by positive regulation of macrophage inflammatory protein-1 gamma production [GO:0071648] Sources: GOC:add, GOC:rv Relationships: is a type of chemokine production [GO:0032602] Definition: The appearance of macrophage inflammatory protein-1 gamma due to biosynthesis or secretion following a cellular stimulus, resulting in an increase in its intracellular or extracellular levels. Also known as: CCL9 production, MIP-1g production, chemokine (C-C motif) ligand 9 production